{
  "gene": "UniProtKB:Q15910",
  "gene_name": "Histone-lysine N-methyltransferase EZH2",
  "gene_symbol": "EZH2",
  "term_id": "GO:0003682",
  "term_label": "chromatin binding"
}